{
  "term_id": "GO:0006357",
  "gene": "UniProtKB:Q96MR9",
  "term_label": "regulation of transcription by RNA polymerase II",
  "gene_symbol": "ZNF560",
  "gene_name": "Zinc finger protein 560"
}